{
  "gene": "UniProtKB:A8MTZ7",
  "gene_name": "Uncharacterized protein C12orf71",
  "gene_symbol": "C12orf71",
  "term_label": "Unknown molecular function",
  "term_id": "UNKNOWN:0001"
}